{
  "gene_symbol": "ABCF1",
  "gene": "UniProtKB:Q8NE71",
  "term_id": "UNKNOWN:0002",
  "gene_name": "ATP-binding cassette sub-family F member 1",
  "term_label": "Unknown biological process"
}